{
  "gene_name": "Probable E3 SUMO-protein ligase RNF212",
  "term_id": "GO:0000795",
  "gene": "UniProtKB:Q495C1",
  "gene_symbol": "RNF212",
  "term_label": "synaptonemal complex"
}